{
  "gene_name": "Cytochrome P450 2A6",
  "gene": "UniProtKB:P11509",
  "term_id": "GO:0006805",
  "gene_symbol": "CYP2A6",
  "term_label": "xenobiotic metabolic process"
}